{
  "gene_symbol": "KEAP1",
  "term_id": "GO:0031463",
  "term_label": "Cul3-RING ubiquitin ligase complex",
  "gene_name": "Kelch-like ECH-associated protein 1",
  "gene": "UniProtKB:Q14145"
}